cellular heat acclimation [GO:0070370] (biological process) Also known as: cellular thermotolerance Relationships: is a type of heat acclimation [GO:0010286]; is a type of cellular response to heat [GO:0034605] Definition: Any process that increases heat tolerance of a cell in response to high temperatures. Sources: GOC:jp